{
  "term_label": "regulation of cell migration",
  "term_id": "GO:0030334",
  "gene_name": "STE20-like serine_threonine-protein kinase",
  "gene": "UniProtKB:Q9H2G2",
  "gene_symbol": "SLK"
}